{
  "term_id": "GO:0005783",
  "term_label": "endoplasmic reticulum",
  "gene_name": "Vesicle transport protein GOT1A",
  "gene": "UniProtKB:Q6ZVE7",
  "gene_symbol": "GOLT1A"
}